{
  "term_id": "GO:0003711",
  "gene_symbol": "EAF1",
  "gene": "UniProtKB:Q96JC9",
  "gene_name": "ELL-associated factor 1",
  "term_label": "transcription elongation factor activity"
}